regulation of flavonol biosynthetic process [GO:1900384] (biological process) Definition: Any process that modulates the frequency, rate or extent of flavonol biosynthetic process. Relationships: is a type of regulation of flavonoid biosynthetic process [GO:0009962]; regulates flavonol biosynthetic process [GO:0051555] Sources: GOC:TermGenie Subtypes: negative regulation of flavonol biosynthetic process [GO:1900385], positive regulation of flavonol biosynthetic process [GO:1900386]